{
  "term_id": "GO:0005634",
  "term_label": "nucleus",
  "gene_symbol": "POLH",
  "gene": "UniProtKB:Q9Y253",
  "gene_name": "DNA polymerase eta"
}